positive regulation of lateral attachment of mitotic spindle microtubules to kinetochore [GO:1905116] (biological process) Definition: Any process that activates or increases the frequency, rate or extent of lateral attachment of mitotic spindle microtubules to kinetochore. References: PMID:22375062 Sources: GOC:TermGenie, GO_REF:0000058 Also known as: up regulation of lateral attachment of mitotic spindle microtubules to kinetochore, up-regulation of lateral attachment of mitotic spindle microtubules to kinetochore, upregulation of lateral attachment of mitotic spindle microtubules to kinetochore, activation of lateral attachment of mitotic spindle microtubules to kinetochore Relationships: is a type of positive regulation of attachment of mitotic spindle microtubules to kinetochore [GO:1902425]; is a type of GO:1905115; positively regulates lateral attachment of mitotic spindle microtubules to kinetochore [GO:0099607]